theta DNA replication [GO:0070582] (biological process) Relationships: is a type of DNA-templated DNA replication [GO:0006261] Also known as: theta replication Definition: A DNA-dependent DNA replication process in which a double-stranded DNA molecule is synthesized from a circular duplex template. Sources: GOC:cb, GOC:mah, ISBN:0198506732